{
  "gene_name": "Transcription intermediary factor 1-beta",
  "gene_symbol": "TRIM28",
  "gene": "UniProtKB:Q13263",
  "term_label": "protein sumoylation",
  "term_id": "GO:0016925"
}